precorrin-3B C17-methyltransferase activity [GO:0030789] (MF) Sources: EC:2.1.1.131 Relationships: is a type of GO:0008757 Definition: Catalysis of the reaction: S-adenosyl-L-methionine + precorrin-3B = S-adenosyl-L-homocysteine + precorrin 4. Also known as: CobJ, S-adenosyl-L-methionine:precorrin-3B C17-methyltransferase activity, precorrin-3 methylase activity, precorrin-3 methyltransferase activity